{
  "gene_symbol": "MYD88",
  "gene_name": "Myeloid differentiation primary response protein MyD88",
  "term_id": "GO:0050830",
  "gene": "UniProtKB:Q99836",
  "term_label": "defense response to Gram-positive bacterium"
}